negative regulation of mesonephric nephron tubule epithelial cell differentiation [GO:2000094] (biological process) Sources: GOC:mtg_kidney_jan10 Definition: Any process that stops, prevents, or reduces the frequency, rate or extent of mesonephric nephron tubule epithelial cell differentiation. Relationships: is a type of negative regulation of nephron tubule epithelial cell differentiation [GO:0072183]; is a type of regulation of mesonephric nephron tubule epithelial cell differentiation [GO:2000093]; negatively regulates GO:0061265